megagametophyte egg cell nucleus [GO:0043082] (cellular component) Relationships: is a type of megasporocyte nucleus [GO:0043076] Definition: The nucleus of a plant egg cell. This nucleus is found at the micropylar end of the embryo. Sources: GOC:jl, GOC:mtg_sensu